{
  "term_label": "signal transduction",
  "gene_symbol": "DUSP15",
  "term_id": "GO:0007165",
  "gene_name": "Dual specificity protein phosphatase 15",
  "gene": "UniProtKB:Q9H1R2"
}